{
  "gene_name": "Eukaryotic translation initiation factor 3 subunit A",
  "gene": "UniProtKB:Q14152",
  "term_label": "eukaryotic translation initiation factor 3 complex, eIF3m",
  "term_id": "GO:0071541",
  "gene_symbol": "EIF3A"
}